{
  "gene_symbol": "KLC2",
  "term_label": "kinesin binding",
  "term_id": "GO:0019894",
  "gene": "UniProtKB:Q9H0B6",
  "gene_name": "Kinesin light chain 2"
}